{
  "gene_symbol": "DIP2A",
  "gene_name": "Disco-interacting protein 2 homolog A",
  "term_id": "GO:0009986",
  "gene": "UniProtKB:Q14689",
  "term_label": "cell surface"
}